{
  "term_label": "retrograde vesicle-mediated transport, Golgi to endoplasmic reticulum",
  "gene_name": "Golgi-specific brefeldin A-resistance guanine nucleotide exchange factor 1",
  "gene_symbol": "GBF1",
  "gene": "UniProtKB:Q92538",
  "term_id": "GO:0006890"
}